{
  "term_label": "fusion of sperm to egg plasma membrane involved in single fertilization",
  "gene_name": "Fertilization-influencing membrane protein",
  "gene_symbol": "FIMP",
  "gene": "UniProtKB:Q96LL3",
  "term_id": "GO:0007342"
}